{
  "term_id": "UNKNOWN:0002",
  "term_label": "Unknown biological process",
  "gene": "UniProtKB:Q6ZRC1",
  "gene_symbol": "C4orf50",
  "gene_name": "Uncharacterized protein C4orf50"
}